Y-form DNA binding [GO:0000403] (molecular function) Definition: Binding to a DNA segment shaped like a Y. This shape occurs when DNA contains a region of paired double-stranded DNA on one end and a region of unpaired DNA strands on the opposite end. References: PMID:16781730 Sources: GOC:elh Also known as: forked DNA binding, splayed Y-form DNA binding Relationships: is a type of DNA secondary structure binding [GO:0000217]